{
  "gene": "UniProtKB:B7ZAQ6",
  "term_label": "intracellular pH reduction",
  "gene_name": "Golgi pH regulator A",
  "gene_symbol": "GPR89A",
  "term_id": "GO:0051452"
}